{
  "term_label": "nucleus",
  "gene": "UniProtKB:Q9NR55",
  "gene_name": "Basic leucine zipper transcriptional factor ATF-like 3",
  "term_id": "GO:0005634",
  "gene_symbol": "BATF3"
}